{
  "gene_name": "Leucine-rich repeat-containing protein 63",
  "term_label": "Unknown molecular function",
  "gene_symbol": "LRRC63",
  "gene": "UniProtKB:Q05C16",
  "term_id": "UNKNOWN:0001"
}